{
  "gene_symbol": "UTP18",
  "term_label": "small-subunit processome",
  "gene": "UniProtKB:Q9Y5J1",
  "gene_name": "U3 small nucleolar RNA-associated protein 18 homolog",
  "term_id": "GO:0032040"
}